epinephrine-mediated vasodilation [GO:0003121] (biological process) Also known as: regulation of vasodilation by adrenaline, regulation of vasodilation by circulating adrenaline, regulation of vasodilation by circulating epinephrine, regulation of vasodilation by epinephrine, regulation of vasodilation by neuronal adrenaline, regulation of vasodilation by neuronal epinephrine Definition: A vasodilation process resulting from secretion of epinephrine into the bloodstream or released by nerve endings. Sources: GOC:mtg_cardio Relationships: is a type of vasodilation [GO:0042311]